foregut regionalization [GO:0060423] (BP) Definition: The pattern specification process that results in the spatial subdivision of an axis or axes along the foregut to define an area or volume in which specific patterns of cell differentiation will take place. Relationships: is a type of GO:0009952 Subtypes: lung field specification [GO:0060424] Sources: GOC:dph, GOC:mtg_lung